{
  "term_label": "Notch signaling pathway",
  "gene_symbol": "NOTCH3",
  "term_id": "GO:0007219",
  "gene_name": "Neurogenic locus notch homolog protein 3",
  "gene": "UniProtKB:Q9UM47"
}